{
  "gene_name": "DNA damage-induced apoptosis suppressor protein",
  "gene": "UniProtKB:Q8IXT1",
  "term_id": "UNKNOWN:0001",
  "term_label": "Unknown molecular function",
  "gene_symbol": "DDIAS"
}